negative regulation of formation of structure involved in a symbiotic process [GO:0044147] (biological process) Note: This term partially replaces the obsolete term 'negative regulation of growth or development of symbiont during interaction with host ; GO:0075340'. Also known as: negative regulation of development of symbiont during interaction with host, negative regulation of development of symbiont involved in interaction with host Subtypes: negative regulation of development of symbiont in host [GO:0044131], GO:0075047, negative regulation of arbuscule formation for nutrient acquisition from host [GO:0075331] Relationships: is a type of modulation of formation of structure involved in a symbiotic process [GO:0044145]; is a type of GO:0048519; RO_0002212 GO:0044111 Sources: GOC:jl, GOC:pamgo_curators Definition: Any process that stops, prevents, or reduces the frequency, rate or extent of the progression of an organism from an initial condition to a later condition, occurring in, on or near the exterior of its host organism.